{
  "gene_name": "Sodium-independent sulfate anion transporter",
  "term_label": "sulfate transmembrane transporter activity",
  "term_id": "GO:0015116",
  "gene_symbol": "SLC26A11",
  "gene": "UniProtKB:Q86WA9"
}